{
  "gene": "UniProtKB:Q6ZTW0",
  "gene_name": "Tubulin polyglutamylase complex subunit 1",
  "term_label": "microtubule organizing center",
  "term_id": "GO:0005815",
  "gene_symbol": "TPGS1"
}